{
  "term_label": "negative regulation of transcription by RNA polymerase II",
  "term_id": "GO:0000122",
  "gene_symbol": "MAGEC1",
  "gene": "UniProtKB:O60732",
  "gene_name": "Melanoma-associated antigen C1"
}